{
  "gene": "UniProtKB:O43396",
  "gene_symbol": "TXNL1",
  "gene_name": "Thioredoxin-like protein 1",
  "term_label": "Unknown biological process",
  "term_id": "UNKNOWN:0002"
}